T cell inhibitory signaling pathway [GO:0002770] (biological process) References: PMID:15258309 Sources: GOC:add Relationships: is a type of immune response-inhibiting cell surface receptor signaling pathway [GO:0002767] Definition: The series of molecular signals initiated by an extracellular ligand binding to a receptor on the surface of a T cell capable of inhibiting an immune effector process contributing to an immune response. Also known as: T cell inhibitory signalling pathway, T lymphocyte inhibitory signaling pathway, T-cell inhibitory signaling pathway, T-lymphocyte inhibitory signaling pathway